{
  "term_label": "Unknown molecular function",
  "gene_symbol": "NPIPA1",
  "gene": "UniProtKB:Q9UND3",
  "gene_name": "Nuclear pore complex-interacting protein family member A1",
  "term_id": "UNKNOWN:0001"
}